{
  "gene_name": "DNA excision repair protein ERCC-6-like",
  "term_label": "DNA repair",
  "gene": "UniProtKB:Q2NKX8",
  "gene_symbol": "ERCC6L",
  "term_id": "GO:0006281"
}